{
  "gene_symbol": "FHDC1",
  "gene_name": "FH2 domain-containing protein 1",
  "gene": "UniProtKB:Q9C0D6",
  "term_id": "GO:0005884",
  "term_label": "actin filament"
}